{
  "gene_symbol": "TRIM73",
  "term_id": "GO:0061630",
  "term_label": "ubiquitin protein ligase activity",
  "gene": "UniProtKB:Q86UV7",
  "gene_name": "Tripartite motif-containing protein 73"
}